{
  "gene_symbol": "CLPSL1",
  "gene": "UniProtKB:A2RUU4",
  "term_id": "UNKNOWN:0003",
  "gene_name": "Colipase-like protein 1",
  "term_label": "Unknown cellular component"
}